{
  "gene": "UniProtKB:Q9Y6I8",
  "gene_name": "Peroxisomal membrane protein 4",
  "term_id": "UNKNOWN:0002",
  "gene_symbol": "PXMP4",
  "term_label": "Unknown biological process"
}